para-aminobenzoic acid metabolic process [GO:0046482] (biological process) Also known as: 4-aminobenzoic acid metabolic process, 4-aminobenzoic acid metabolism, PABA metabolic process, PABA metabolism, p-aminobenzoic acid metabolic process, p-aminobenzoic acid metabolism, para-aminobenzoic acid metabolism, vitamin Bx metabolic process, vitamin Bx metabolism Relationships: is a type of aromatic amino acid metabolic process [GO:0009072]; is_a monocarboxylic acid metabolic process [GO:0032787]; is a type of benzene-containing compound metabolic process [GO:0042537] References: PMID:11377864, PMID:11960743 Sources: ISBN:0198506732 Definition: The chemical reactions and pathways involving para-aminobenzoic acid, an intermediate in the synthesis of folic acid, a compound which some organisms, e.g. prokaryotes, eukaryotic microbes, and plants, can synthesize de novo. Others, notably mammals, cannot. In yeast, it is present as a factor in the B complex of vitamins. Subtypes: 4-aminobenzoate biosynthetic process [GO:0008153]